{
  "term_label": "Unknown cellular component",
  "gene_symbol": "NR2F1",
  "gene": "UniProtKB:P10589",
  "term_id": "UNKNOWN:0003",
  "gene_name": "COUP transcription factor 1"
}